{
  "gene": "UniProtKB:Q9Y4C0",
  "gene_name": "Neurexin-3",
  "term_id": "GO:0007612",
  "gene_symbol": "NRXN3",
  "term_label": "learning"
}